{
  "term_label": "Unknown molecular function",
  "gene": "UniProtKB:A6NDY2",
  "gene_symbol": "FAM90A10",
  "term_id": "UNKNOWN:0001",
  "gene_name": "Putative protein FAM90A10"
}